{
  "gene_symbol": "PER2",
  "term_id": "GO:0000976",
  "gene_name": "Period circadian protein homolog 2",
  "term_label": "transcription cis-regulatory region binding",
  "gene": "UniProtKB:O15055"
}